{
  "gene": "UniProtKB:Q9NPF5",
  "gene_symbol": "DMAP1",
  "term_id": "GO:0000122",
  "term_label": "negative regulation of transcription by RNA polymerase II",
  "gene_name": "DNA methyltransferase 1-associated protein 1"
}